positive regulation of replicative senescence [GO:1904728] (biological process) Relationships: is a type of GO:0090068; is a type of GO:1904726; RO_0002213 replicative senescence [GO:0090399] Also known as: up regulation of replicative senescence, up-regulation of replicative senescence, upregulation of replicative senescence, activation of replicative senescence Definition: Any process that activates or increases the frequency, rate or extent of replicative senescence. References: PMID:23496142 Sources: GOC:BHF, GOC:BHF_miRNA, GOC:TermGenie, GOC:rph, GO_REF:0000058